synaptic ribbon [GO:0098681] (cellular component) Definition: A non-membrane bound, electron dense structure associated that extends perpendicular to the presynaptic membrane in ribbon synapses. The ribbon's surface is studded with small particles to which synaptic vesicles tether via fine filaments. The tethered vesicles function as a pool, several fold greater than the docked pool available for fast release, which supports sustained release of vesicles. Synaptic ribbons may be plate like or spherical. Relationships: is a type of intracellular membraneless organelle [GO:0043232] References: PMID:15626493